{
  "gene_name": "Arginase-2, mitochondrial",
  "term_label": "urea cycle",
  "gene": "UniProtKB:P78540",
  "gene_symbol": "ARG2",
  "term_id": "GO:0000050"
}